initiation of appressorium formation [GO:0075025] (biological process) Definition: The process in which a relatively unspecialized cell starts to acquire specialized features of the symbiont appressorium to aid in infection of the host. The host is defined as the larger of the organisms involved in a symbiotic interaction. Relationships: is a type of formation of structure involved in a symbiotic process [GO:0044111]; is part of appressorium formation [GO:0075016] Note: Note that this term should not be used to annotate gene products of the host. It should only be used to annotate those gene products from the symbiont involved in this process. Also known as: appressorium initiation on or near host, initiation of appressorium by symbiont on or near host, initiation of symbiont appressorium on or near host, initiation of appressorium on or near host Sources: GOC:pamgo_curators